{
  "gene_name": "Electrogenic sodium bicarbonate cotransporter 1",
  "gene": "UniProtKB:Q9Y6R1",
  "term_id": "GO:0005886",
  "gene_symbol": "SLC4A4",
  "term_label": "plasma membrane"
}